{
  "term_label": "regulation of JNK cascade",
  "gene_name": "MyoD family inhibitor",
  "gene": "UniProtKB:Q99750",
  "gene_symbol": "MDFI",
  "term_id": "GO:0046328"
}